axon extension involved in axon guidance [GO:0048846] (biological process) Sources: GOC:ef, GOC:jid Relationships: is a type of GO:0048675; is_a GO:1902284; is part of axon guidance [GO:0007411] Regulation: regulated by regulation of axon extension involved in axon guidance [GO:0048841]; positively regulated by GO:0048842; negatively regulated by negative regulation of axon extension involved in axon guidance [GO:0048843] Definition: The long distance growth of a single cell process, that is involved in the migration of an axon growth cone, where the migration is directed to a specific target site by a combination of attractive and repulsive cues.